{
  "term_label": "chromatin binding",
  "gene_symbol": "SET",
  "gene_name": "Protein SET",
  "term_id": "GO:0003682",
  "gene": "UniProtKB:Q01105"
}